isopentenyl adenine catabolic process [GO:0034266] (biological process) Also known as: isopentenyl adenine breakdown, isopentenyl adenine catabolism, isopentenyl adenine degradation, isopentenyladenine catabolic process Definition: The chemical reactions and pathways resulting in the breakdown of the cytokinin 6-isopentenyladenine. Relationships: is a type of GO:0009823; is a type of purine-containing compound catabolic process [GO:0072523] References: PMID:18216168 Sources: GOC:mah